{
  "gene": "UniProtKB:Q07812",
  "term_id": "GO:0005741",
  "gene_symbol": "BAX",
  "gene_name": "Apoptosis regulator BAX",
  "term_label": "mitochondrial outer membrane"
}